{
  "term_id": "GO:0045109",
  "gene": "UniProtKB:Q9NSB2",
  "gene_symbol": "KRT84",
  "gene_name": "Keratin, type II cuticular Hb4",
  "term_label": "intermediate filament organization"
}